{
  "gene": "UniProtKB:Q15771",
  "gene_symbol": "RAB30",
  "term_label": "vesicle-mediated transport",
  "term_id": "GO:0016192",
  "gene_name": "Ras-related protein Rab-30"
}